{
  "gene_symbol": "TWF2",
  "gene_name": "Twinfilin-2",
  "term_label": "actin monomer binding",
  "term_id": "GO:0003785",
  "gene": "UniProtKB:Q6IBS0"
}